{
  "gene_name": "Immunoglobulin heavy variable 3_OR16-17 (non-functional) (Fragment)",
  "term_id": "GO:0016064",
  "gene": "UniProtKB:S4R3C0",
  "term_label": "immunoglobulin mediated immune response",
  "gene_symbol": "IGHV3OR16-17"
}